{
  "term_id": "GO:0006979",
  "term_label": "response to oxidative stress",
  "gene": "UniProtKB:P30519",
  "gene_name": "Heme oxygenase 2",
  "gene_symbol": "HMOX2"
}